{
  "term_id": "GO:0003858",
  "gene": "UniProtKB:Q9BUT1",
  "term_label": "3-hydroxybutyrate dehydrogenase activity",
  "gene_name": "Dehydrogenase_reductase SDR family member 6",
  "gene_symbol": "BDH2"
}